{
  "term_label": "Unknown cellular component",
  "gene": "UniProtKB:Q8IYB0",
  "gene_symbol": "Q8IYB0",
  "term_id": "UNKNOWN:0003",
  "gene_name": "Putative uncharacterized protein MGC39545"
}